indole acetic acid carboxyl methyltransferase activity [GO:0051749] (molecular function) Relationships: is a type of methyltransferase activity [GO:0008168] Definition: Catalysis of the reaction: indole acetic acid + S-adenosyl-methionine = methyl indole acetic acid ester + S-adenosyl-homocysteine. Also known as: IAA carboxyl methyltransferase activity References: PMID:16169896